negative regulation of protein deubiquitination [GO:0090086] (biological process) Relationships: is a type of regulation of protein deubiquitination [GO:0090085]; is a type of negative regulation of protein modification by small protein conjugation or removal [GO:1903321]; negatively regulates protein deubiquitination [GO:0016579] Sources: GOC:BHF, GOC:dph, GOC:tb Definition: Any process that decreases the frequency, rate or extent of protein deubiquitination. Protein deubiquitination is the removal of one or more ubiquitin groups from a protein. Subtypes: negative regulation of protein K63-linked deubiquitination [GO:1903005], negative regulation of protein K48-linked deubiquitination [GO:1903094]